{
  "gene_symbol": "CLEC14A",
  "term_label": "extracellular matrix binding",
  "term_id": "GO:0050840",
  "gene_name": "C-type lectin domain family 14 member A",
  "gene": "UniProtKB:Q86T13"
}